{
  "term_id": "UNKNOWN:0001",
  "gene": "UniProtKB:Q499Z3",
  "term_label": "Unknown molecular function",
  "gene_name": "Schlafen-like protein 1",
  "gene_symbol": "SLFNL1"
}